positive regulation of myoblast differentiation [GO:0045663] (BP) Relationships: is_a positive regulation of cell differentiation [GO:0045597]; is a type of regulation of myoblast differentiation [GO:0045661]; positively regulates myoblast differentiation [GO:0045445] Subtypes: positive regulation of cardiac muscle cell myoblast differentiation [GO:2000700] Sources: CL:0000056, GOC:go_curators, GOC:mtg_muscle Also known as: up regulation of myoblast differentiation, up-regulation of myoblast differentiation, upregulation of myoblast differentiation, activation of myoblast differentiation, stimulation of myoblast differentiation Definition: Any process that activates or increases the frequency, rate or extent of myoblast differentiation. A myoblast is a mononucleate cell type that, by fusion with other myoblasts, gives rise to the myotubes that eventually develop into skeletal muscle fibers.